intermediate mesoderm formation [GO:0048391] (biological process) Sources: GOC:dgh Definition: The process that gives rise to the intermediate mesoderm. This process pertains to the initial formation of the structure from unspecified parts. Relationships: is a type of mesoderm formation [GO:0001707]; is part of intermediate mesoderm morphogenesis [GO:0048390]